post-embryonic appendage morphogenesis [GO:0035120] (biological process) Sources: ISBN:0582227089 Definition: The process, occurring after embryonic development, by which the anatomical structures of an appendage are generated and organized. An appendage is an organ or part that is attached to the trunk of an organism, such as a limb or a branch. Subtypes: GO:0007476, imaginal disc-derived leg morphogenesis [GO:0007480], post-embryonic limb morphogenesis [GO:0035127], post-embryonic pectoral fin morphogenesis [GO:0035130], GO:0035131, GO:0035132, haltere morphogenesis [GO:0048735] Relationships: is a type of post-embryonic animal morphogenesis [GO:0009886]; is a type of appendage morphogenesis [GO:0035107]